cellular response to vanadate(3-) [GO:1902439] (biological process) Definition: Any process that results in a change in state or activity of a cell (in terms of movement, secretion, enzyme production, gene expression, etc.) as a result of a vanadate(3-) stimulus. References: PMID:7489911 Sources: GOC:TermGenie, GOC:di Relationships: is a type of cellular response to oxygen-containing compound [GO:1901701]; is a type of GO:1902438